simple leaf morphogenesis [GO:0060776] (biological process) Relationships: is a type of leaf morphogenesis [GO:0009965] Definition: The leaf morphogenesis process which results in the shaping of a simple leaf. A simple leaf is a leaf in which the lamina is undivided. Sources: GOC:dph, GOC:sdb_2009, GOC:tb